{
  "term_id": "UNKNOWN:0001",
  "term_label": "Unknown molecular function",
  "gene": "UniProtKB:Q9BVV7",
  "gene_name": "Mitochondrial import inner membrane translocase subunit Tim21",
  "gene_symbol": "TIMM21"
}